miRNA inhibitor activity via base-pairing [GO:0140869] (molecular function) References: PMID:34454184 Also known as: miRNA inhibitor activity, miRNA binding involved in posttranscriptional gene silencing, miRNA base-pairing repressor activity, miRNA sponge, base-pairing target-directed miRNA suppressor activity, base-pairing target-directed microRNA suppressor activity Definition: Stops, prevents or reduces the activity of miRNA-mediated gene silencing activity by base-pairing with a target miRNA. An example of this activity is mediated by long non-coding RNAs (lncRNAs). Note: This term is intended for regulatory non-coding RNAs that act by base-pairing with a target microRNA. Relationships: is a type of GO:0035198; is a type of molecular function inhibitor activity [GO:0140678]